{
  "gene_symbol": "HPCA",
  "term_label": "regulation of signal transduction",
  "gene_name": "Neuron-specific calcium-binding protein hippocalcin",
  "term_id": "GO:0009966",
  "gene": "UniProtKB:P84074"
}